{
  "gene_symbol": "TMBIM1",
  "gene": "UniProtKB:Q969X1",
  "gene_name": "Protein lifeguard 3",
  "term_id": "GO:1902042",
  "term_label": "negative regulation of extrinsic apoptotic signaling pathway via death domain receptors"
}